inositol trisphosphate biosynthetic process [GO:0032959] (BP) Also known as: IP3 biosynthesis, IP3 biosynthetic process, inositol trisphosphate anabolism, inositol trisphosphate biosynthesis, inositol trisphosphate formation, inositol trisphosphate synthesis, myo-inositol trisphosphate biosynthetic process Sources: GOC:mah Regulation: regulated by regulation of inositol trisphosphate biosynthetic process [GO:0032960]; RO_0002212 by GO:0032961; positively regulated by positive regulation of inositol trisphosphate biosynthetic process [GO:0032962] Definition: The chemical reactions and pathways resulting in the formation of inositol trisphosphate, 1,2,3,4,5,6-cyclohexanehexol, with three phosphate groups attached. Relationships: is a type of GO:0032957; is a type of inositol phosphate biosynthetic process [GO:0032958]